{
  "gene_symbol": "USPL1",
  "term_label": "Cajal body",
  "gene": "UniProtKB:Q5W0Q7",
  "gene_name": "SUMO-specific isopeptidase USPL1",
  "term_id": "GO:0015030"
}